dentate gyrus mossy fiber [GO:0044302] (cellular component) References: PMID:17765709 Sources: NIF_Subcellular:nlx_subcell_20090601 Definition: Hippocampal mossy fiber produced by dentate gyrus granule cells. Also known as: granule cell axon, dentate gyrus mossy fibre Relationships: is a type of hippocampal mossy fiber [GO:0097457]